{
  "gene_name": "Glomulin",
  "term_id": "GO:0005737",
  "gene": "UniProtKB:Q92990",
  "term_label": "cytoplasm",
  "gene_symbol": "GLMN"
}